lumenal side of smooth endoplasmic reticulum membrane [GO:0098558] (cellular component) Sources: GOC:ab, GOC:dos Definition: The side (leaflet) of the smooth endoplasmic reticulum membrane that faces the lumen. Relationships: is a type of lumenal side of endoplasmic reticulum membrane [GO:0098553]; is part of GO:0030868